{
  "gene_symbol": "ZFP28",
  "term_label": "RNA polymerase II cis-regulatory region sequence-specific DNA binding",
  "gene_name": "Zinc finger protein 28 homolog",
  "term_id": "GO:0000978",
  "gene": "UniProtKB:Q8NHY6"
}